{
  "gene": "UniProtKB:Q01082",
  "gene_name": "Spectrin beta chain, non-erythrocytic 1",
  "term_id": "GO:0051015",
  "term_label": "actin filament binding",
  "gene_symbol": "SPTBN1"
}